{
  "term_id": "UNKNOWN:0002",
  "gene_symbol": "SNTB2",
  "gene": "UniProtKB:Q13425",
  "term_label": "Unknown biological process",
  "gene_name": "Beta-2-syntrophin"
}